{
  "term_id": "UNKNOWN:0003",
  "gene_name": "Leucine-rich repeat, immunoglobulin-like domain and transmembrane domain-containing protein 3",
  "term_label": "Unknown cellular component",
  "gene_symbol": "LRIT3",
  "gene": "UniProtKB:Q3SXY7"
}